pyruvate kinase complex [GO:1902912] (cellular component) Subtypes: PKM2 pyruvate kinase complex [GO:1990361] Definition: A protein complex which is capable of pyruvate kinase activity. Relationships: is a type of GO:0061695 References: PMID:24606918 Sources: GOC:TermGenie, GOC:bhm, GO_REF:0000088 Note: An example of this is PKM2 in human (P14618) in PMID:24606918 (inferred from direct assay).